{
  "gene": "UniProtKB:Q8N1G4",
  "term_label": "phenylalanine-tRNA ligase activity",
  "gene_name": "Leucine-rich repeat-containing protein 47",
  "gene_symbol": "LRRC47",
  "term_id": "GO:0004826"
}